cardiocyte differentiation [GO:0035051] (biological process) Definition: The process in which a relatively unspecialized cell acquires the specialized structural and/or functional features of a cell that will form part of the cardiac organ of an individual. Relationships: is a type of cell differentiation [GO:0030154]; is part of GO:0007507 Sources: GOC:bf Also known as: cardiac cell differentiation, heart cell differentiation Subtypes: cardiac septum cell differentiation [GO:0003292], heart valve cell differentiation [GO:0003293], cardiac endothelial cell differentiation [GO:0003348], cardioblast differentiation [GO:0010002], GO:0055007, cardiac fibroblast cell differentiation [GO:0060935], cardiac neuron differentiation [GO:0060945], cardiac vascular smooth muscle cell differentiation [GO:0060947], cardiac glial cell differentiation [GO:0060950], cardiac neural crest cell differentiation involved in heart development [GO:0061307], endocardial cushion cell differentiation [GO:0061443] Regulation: RO_0002211 by regulation of cardiocyte differentiation [GO:1905207]; negatively regulated by negative regulation of cardiocyte differentiation [GO:1905208]; positively regulated by positive regulation of cardiocyte differentiation [GO:1905209]